{
  "gene_symbol": "Q1RN00",
  "term_label": "Unknown cellular component",
  "gene_name": "Putative uncharacterized protein LOC151760",
  "term_id": "UNKNOWN:0003",
  "gene": "UniProtKB:Q1RN00"
}